DNA dealkylation [GO:0035510] (biological process) Definition: The removal of an alkyl group from one or more nucleotides within an DNA molecule. Relationships: is a type of DNA modification [GO:0006304] Sources: GOC:bf